septin collar organization [GO:0140544] (biological process) Also known as: cellular bud neck septin hourglass organization Definition: A process that is carried out at the cellular level which results in the assembly, arrangement of constituent parts, or disassembly of cytoskeletal structures comprising the septin collar. References: PMID:21736496, PMID:32386534 Relationships: is a type of septin cytoskeleton organization [GO:0032185]